mevastatin biosynthetic process [GO:0140877] (biological process) Relationships: is a type of polyketide biosynthetic process [GO:0030639]; is a type of mycotoxin biosynthetic process [GO:0043386]; is a type of lactone biosynthetic process [GO:1901336] Also known as: mevastatin anabolism, mevastatin biosynthesis, mevastatin formation, mevastatin synthesis Definition: The chemical reactions and pathways resulting in the formation of mevastatin , also known as compactin or ML-236B, and which acts as a potent competitive inhibitor of HMG-CoA reductase. References: PMID:12172803, PMID:12242508